inositol 3-methyltransferase activity [GO:0030740] (molecular function) Relationships: is a type of S-adenosylmethionine-dependent methyltransferase activity [GO:0008757] Sources: EC:2.1.1.39, RHEA:18877 Definition: Catalysis of the reaction: S-adenosyl-L-methionine(1+) + myo-inositol = 1D-3-O-methyl-myo-inositol + S-adenosyl-L-homocysteine + H+. Also known as: S-adenosyl-L-methionine:1D-myo-inositol 3-O-methyltransferase activity, S-adenosyl-L-methionine:myo-inositol 1-O-methyltransferase activity, S-adenosylmethionine:myo-inositol 1-methyltransferase activity, inositol L-1-methyltransferase activity, myo-inositol 1-O-methyltransferase (name based on 1L-numbering system and not 1D-numbering), myo-inositol 1-O-methyltransferase activity, myo-inositol 1-methyltransferase activity